{
  "gene_symbol": "RAB3B",
  "term_id": "GO:0031489",
  "term_label": "myosin V binding",
  "gene_name": "Ras-related protein Rab-3B",
  "gene": "UniProtKB:P20337"
}